{
  "gene_name": "Testis-specific serine_threonine-protein kinase 1",
  "term_label": "Unknown cellular component",
  "gene_symbol": "TSSK1B",
  "term_id": "UNKNOWN:0003",
  "gene": "UniProtKB:Q9BXA7"
}